{
  "term_label": "Unknown molecular function",
  "gene": "UniProtKB:A0A0A0MT92",
  "gene_name": "Immunoglobulin lambda joining 7 (Fragment)",
  "gene_symbol": "IGLJ7",
  "term_id": "UNKNOWN:0001"
}